{
  "term_label": "ubiquitin protein ligase binding",
  "gene_name": "Microtubule-associated proteins 1A_1B light chain 3 beta 2",
  "gene": "UniProtKB:A6NCE7",
  "term_id": "GO:0031625",
  "gene_symbol": "MAP1LC3B2"
}